archaeal-type flagellum [GO:0097589] (cellular component) Definition: A non-membrane-bounded organelle superficially similar to a bacterial-type flagellum; they both consist of filaments extending outside the cell, and rotate to propel the cell, but the archaeal flagella (also called archaella) have a unique structure which lacks a central channel. Similar to bacterial type IV pilins, the archaeal flagellins (archaellins) are made with class 3 signal peptides and they are processed by a type IV prepilin peptidase-like enzyme. The archaellins are typically modified by the addition of N-linked glycans which are necessary for proper assembly and/or function. References: PMID:21265748, PMID:23146836, PMID:23204365, PMID:24330313 Sources: GOC:cilia, GOC:krc, Wikipedia:Flagellum#Archaeal Relationships: is a type of cell projection [GO:0042995]; is a type of membraneless organelle [GO:0043228] Also known as: archaellum, archaeal flagellum, archaella